{
  "gene_symbol": "PIK3C2A",
  "term_label": "1-phosphatidylinositol-3-kinase activity",
  "term_id": "GO:0016303",
  "gene": "UniProtKB:O00443",
  "gene_name": "Phosphatidylinositol 4-phosphate 3-kinase C2 domain-containing subunit alpha"
}